{
  "gene": "UniProtKB:Q8N9I5",
  "term_label": "oxidoreductase activity, acting on paired donors, with oxidation of a pair of donors resulting in the reduction of molecular oxygen to two molecules of water",
  "term_id": "GO:0016717",
  "gene_symbol": "FADS6",
  "gene_name": "Fatty acid desaturase 6"
}